{
  "term_label": "ubiquitin protein ligase activity",
  "term_id": "GO:0061630",
  "gene_symbol": "TRIM14",
  "gene_name": "Tripartite motif-containing protein 14",
  "gene": "UniProtKB:Q14142"
}